endothelial cell migration [GO:0043542] (biological process) Regulation: regulated by GO:0010594; positively regulated by positive regulation of endothelial cell migration [GO:0010595]; negatively regulated by GO:0010596 Sources: GOC:go_curators Relationships: is a type of cell migration [GO:0016477] Definition: The orderly movement of an endothelial cell into the extracellular matrix to form an endothelium. Subtypes: GO:0035767, blood vessel endothelial cell migration [GO:0043534], GO:1904977